{
  "gene_symbol": "OR2AP1",
  "gene_name": "Olfactory receptor 2AP1",
  "term_label": "olfactory receptor activity",
  "term_id": "GO:0004984",
  "gene": "UniProtKB:Q8NGE2"
}